regulation of heart rate by cardiac conduction [GO:0086091] (biological process) Relationships: is a type of regulation of heart rate [GO:0002027]; is a type of cardiac conduction [GO:0061337] Definition: A cardiac conduction process that modulates the frequency or rate of heart contraction. Sources: GOC:BHF, GOC:mtg_cardiac_conduct_nov11